{
  "gene_name": "Glycophorin-C",
  "term_id": "UNKNOWN:0001",
  "gene": "UniProtKB:P04921",
  "term_label": "Unknown molecular function",
  "gene_symbol": "GYPC"
}